{
  "gene_name": "Bis(5'-adenosyl)-triphosphatase",
  "term_label": "cytoplasm",
  "gene_symbol": "FHIT",
  "term_id": "GO:0005737",
  "gene": "UniProtKB:P49789"
}